{
  "gene_symbol": "SPATA2L",
  "term_label": "Unknown biological process",
  "gene_name": "Spermatogenesis-associated protein 2-like protein",
  "gene": "UniProtKB:Q8IUW3",
  "term_id": "UNKNOWN:0002"
}